{
  "term_label": "early endosome",
  "gene_symbol": "RUBCN",
  "gene_name": "Run domain Beclin-1-interacting and cysteine-rich domain-containing protein",
  "term_id": "GO:0005769",
  "gene": "UniProtKB:Q92622"
}